{
  "term_id": "GO:0000122",
  "term_label": "negative regulation of transcription by RNA polymerase II",
  "gene": "UniProtKB:Q96T92",
  "gene_name": "Insulinoma-associated protein 2",
  "gene_symbol": "INSM2"
}